{
  "gene_name": "Protein IMPACT",
  "term_id": "GO:0140469",
  "term_label": "GCN2-mediated signaling",
  "gene": "UniProtKB:Q9P2X3",
  "gene_symbol": "IMPACT"
}